{
  "gene": "UniProtKB:O43324",
  "gene_name": "Eukaryotic translation elongation factor 1 epsilon-1",
  "term_id": "GO:0005737",
  "term_label": "cytoplasm",
  "gene_symbol": "EEF1E1"
}